positive regulation of homoserine biosynthetic process [GO:1901712] (biological process) Definition: Any process that activates or increases the frequency, rate or extent of homoserine biosynthetic process. Relationships: is a type of positive regulation of small molecule metabolic process [GO:0062013]; is a type of regulation of homoserine biosynthetic process [GO:1901710]; is a type of GO:2000284; positively regulates homoserine biosynthetic process [GO:0009090] Sources: GOC:TermGenie Also known as: activation of homoserine anabolism, activation of homoserine biosynthesis, activation of homoserine formation, activation of homoserine synthesis, positive regulation of homoserine anabolism, positive regulation of homoserine biosynthesis, positive regulation of homoserine formation, positive regulation of homoserine synthesis, up regulation of homoserine anabolism, up regulation of homoserine biosynthesis, up regulation of homoserine biosynthetic process, up regulation of homoserine formation, up regulation of homoserine synthesis, up-regulation of homoserine anabolism, up-regulation of homoserine biosynthesis, up-regulation of homoserine biosynthetic process, up-regulation of homoserine formation, up-regulation of homoserine synthesis, upregulation of homoserine anabolism, upregulation of homoserine biosynthesis, upregulation of homoserine biosynthetic process, upregulation of homoserine formation, upregulation of homoserine synthesis, activation of homoserine biosynthetic process